primary amine secretion [GO:0061531] (biological process) Relationships: is a type of amine transport [GO:0015837]; is_a secretion by cell [GO:0032940] Definition: The regulated release of a primary amine by a cell. Subtypes: primary amine secretion, neurotransmission [GO:0061532], tyramine secretion [GO:0061545] Sources: GOC:dph